{
  "gene_name": "Tubulin beta-2B chain",
  "gene_symbol": "TUBB2B",
  "term_label": "cytoplasm",
  "gene": "UniProtKB:Q9BVA1",
  "term_id": "GO:0005737"
}